{
  "gene_name": "RIMS-binding protein 3B",
  "term_label": "manchette",
  "term_id": "GO:0002177",
  "gene": "UniProtKB:A6NNM3",
  "gene_symbol": "RIMBP3B"
}